{
  "gene": "UniProtKB:B2RBV5",
  "gene_symbol": "MRFAP1L2",
  "term_label": "Unknown biological process",
  "gene_name": "MORF4 family associated protein 1 like 2",
  "term_id": "UNKNOWN:0002"
}